{
  "term_label": "Unknown cellular component",
  "gene_name": "Fibronectin type III domain-containing protein 8",
  "gene_symbol": "FNDC8",
  "gene": "UniProtKB:Q8TC99",
  "term_id": "UNKNOWN:0003"
}